{
  "gene_name": "Putative uncharacterized protein CDRT15P3",
  "gene_symbol": "CDRT15P3",
  "gene": "UniProtKB:P0DPF6",
  "term_id": "UNKNOWN:0001",
  "term_label": "Unknown molecular function"
}